{
  "term_label": "adherens junction",
  "gene_symbol": "CTNNA2",
  "term_id": "GO:0005912",
  "gene": "UniProtKB:P26232",
  "gene_name": "Catenin alpha-2"
}